neural plate regionalization [GO:0060897] (biological process) Sources: GOC:dph, GOC:sdb_2009, GOC:tb Definition: The pattern specification process that results in the subdivision of an axis or axes of the neural plate in space to define an area or volume in which specific patterns of cell differentiation will take place or in which cells interpret a specific environment. Relationships: is a type of GO:0003002; is a type of neural plate pattern specification [GO:0060896] Subtypes: neural plate mediolateral regionalization [GO:0021998], neural plate anterior/posterior regionalization [GO:0021999]